{
  "gene_name": "Vascular endothelial growth factor D",
  "term_id": "GO:0048010",
  "term_label": "vascular endothelial growth factor receptor signaling pathway",
  "gene": "UniProtKB:O43915",
  "gene_symbol": "VEGFD"
}